{
  "gene_symbol": "SLIRP",
  "term_label": "Unknown biological process",
  "gene": "UniProtKB:Q9GZT3",
  "term_id": "UNKNOWN:0002",
  "gene_name": "SRA stem-loop-interacting RNA-binding protein, mitochondrial"
}